{
  "gene_name": "Putative speedy protein E16",
  "gene_symbol": "SPDYE16",
  "gene": "UniProtKB:A6NNV3",
  "term_label": "Unknown biological process",
  "term_id": "UNKNOWN:0002"
}